{
  "gene_name": "HAUS augmin-like complex subunit 8",
  "gene_symbol": "HAUS8",
  "term_label": "spindle assembly",
  "gene": "UniProtKB:Q9BT25",
  "term_id": "GO:0051225"
}